{
  "gene_symbol": "SLC2A1",
  "term_label": "apical plasma membrane",
  "term_id": "GO:0016324",
  "gene": "UniProtKB:P11166",
  "gene_name": "Solute carrier family 2, facilitated glucose transporter member 1"
}